{
  "gene": "UniProtKB:Q02846",
  "term_label": "photoreceptor outer segment membrane",
  "gene_symbol": "GUCY2D",
  "term_id": "GO:0042622",
  "gene_name": "Retinal guanylyl cyclase 1"
}